maintenance of mitotic sister chromatid cohesion, centromeric [GO:0071960] (biological process) Definition: The process in which the association between sister chromatids of a replicated chromosome along the length of the centromeric region is maintained as chromosomes condense, attach to the spindle in a bipolar orientation, and congress to the metaphase plate during a mitotic cell cycle. References: PMID:1708436 Sources: GOC:mah Also known as: maintenance of centromeric mitotic sister chromatin cohesion, maintenance of mitotic sister chromatin cohesion at centromere, maintenance of sister chromatin cohesion at centromere at mitosis Relationships: is_a maintenance of mitotic sister chromatid cohesion [GO:0034088]; is part of mitotic sister chromatid cohesion, centromeric [GO:0071962] Regulation: RO_0002211 by regulation of maintenance of mitotic sister chromatid cohesion, centromeric [GO:2000718]; negatively regulated by negative regulation of maintenance of mitotic sister chromatid cohesion, centromeric [GO:2000719]; positively regulated by GO:2000720